{
  "term_label": "phosphotyrosine residue binding",
  "gene_symbol": "SAMSN1",
  "gene": "UniProtKB:Q9NSI8",
  "gene_name": "SAM domain-containing protein SAMSN-1",
  "term_id": "GO:0001784"
}